mammary stem cell proliferation [GO:0002174] (biological process) Regulation: regulated by regulation of mammary stem cell proliferation [GO:2000101]; negatively regulated by negative regulation of mammary stem cell proliferation [GO:2000102]; positively regulated by positive regulation of mammary stem cell proliferation [GO:2000103] Relationships: is a type of GO:0008283; is part of mammary gland development [GO:0030879] Definition: The expansion of a mammary stem cell population by cell division. Mammary stem cells are a source of cells for growth of the mammary gland during puberty and gestation. These cells can give rise to both the luminal and myoepithelial cell types of the gland, and can regenerate the entire organ. References: PMID:15987436